regulation of prostaglandin secretion [GO:0032306] (biological process) Subtypes: negative regulation of prostaglandin secretion [GO:0032307], positive regulation of prostaglandin secretion [GO:0032308], regulation of fever generation by regulation of prostaglandin secretion [GO:0071810] Sources: GOC:mah Relationships: is a type of regulation of icosanoid secretion [GO:0032303]; is a type of regulation of secretion by cell [GO:1903530]; regulates prostaglandin secretion [GO:0032310] Also known as: regulation of prostacyclin secretion Definition: Any process that modulates the frequency, rate or extent of the regulated release of a prostaglandin from a cell.